CD4-positive or CD8-positive, alpha-beta T cell lineage commitment [GO:0043369] (biological process) Definition: The process in which an immature T cell commits to CD4-positive T cell lineage or the CD8-positive lineage of alpha-beta T cells. Subtypes: CD4-positive, alpha-beta T cell lineage commitment [GO:0043373], GO:0043375 Relationships: is a type of T cell lineage commitment [GO:0002360]; BFO_0000050 positive T cell selection [GO:0043368] Also known as: CD4-positive or CD8-positive, alpha-beta T lymphocyte lineage commitment, CD4-positive or CD8-positive, alpha-beta T-cell lineage commitment, CD4-positive or CD8-positive, alpha-beta T-lymphocyte lineage commitment, CD4-positive/CD8-positive, alpha-beta T cell lineage commitment Sources: ISBN:0781735149